{
  "term_label": "Golgi membrane",
  "term_id": "GO:0000139",
  "gene_name": "Golgi apparatus membrane protein TVP23 homolog B",
  "gene_symbol": "TVP23B",
  "gene": "UniProtKB:Q9NYZ1"
}